{
  "gene_name": "SRC kinase signaling inhibitor 1",
  "gene": "UniProtKB:Q9C0H9",
  "term_id": "GO:0061001",
  "term_label": "regulation of dendritic spine morphogenesis",
  "gene_symbol": "SRCIN1"
}